BMP receptor complex [GO:0070724] (cellular component) Definition: A protein complex that acts as a receptor for bone morphogenetic proteins (BMPs); a homo- or heterodimer of type I and/or type II BMP receptor subunits. Also known as: bone morphogenetic protein receptor complex Relationships: is a type of plasma membrane signaling receptor complex [GO:0098802] References: PMID:19377468 Sources: GOC:mah, GOC:mh